{
  "gene_symbol": "CASP10",
  "term_id": "GO:0043525",
  "gene": "UniProtKB:Q92851",
  "term_label": "positive regulation of neuron apoptotic process",
  "gene_name": "Caspase-10"
}